luteinizing hormone secretion [GO:0032275] (biological process) Sources: ISBN:0198506732 Relationships: is a type of GO:0032274 Definition: The regulated release of luteinizing hormone, a gonadotropic glycoprotein hormone secreted by the anterior pituitary. Regulation: regulated by regulation of luteinizing hormone secretion [GO:0033684]; negatively regulated by negative regulation of luteinizing hormone secretion [GO:0033685]; positively regulated by positive regulation of luteinizing hormone secretion [GO:0033686]